{
  "gene_name": "Aprataxin and PNK-like factor",
  "term_id": "GO:0003906",
  "gene_symbol": "APLF",
  "term_label": "DNA-(apurinic or apyrimidinic site) endonuclease activity",
  "gene": "UniProtKB:Q8IW19"
}